{
  "gene_symbol": "BPI",
  "gene": "UniProtKB:P17213",
  "term_label": "lipopolysaccharide-mediated signaling pathway",
  "gene_name": "Bactericidal permeability-increasing protein",
  "term_id": "GO:0031663"
}